{
  "gene": "UniProtKB:Q13085",
  "term_id": "GO:0005739",
  "term_label": "mitochondrion",
  "gene_symbol": "ACACA",
  "gene_name": "Acetyl-CoA carboxylase 1"
}